{
  "term_label": "regulation of transcription by RNA polymerase II",
  "gene": "UniProtKB:Q9UJW8",
  "gene_name": "Zinc finger protein 180",
  "term_id": "GO:0006357",
  "gene_symbol": "ZNF180"
}